{
  "term_label": "voltage-gated sodium channel activity",
  "gene_symbol": "SCN11A",
  "term_id": "GO:0005248",
  "gene": "UniProtKB:Q9UI33",
  "gene_name": "Sodium channel protein type 11 subunit alpha"
}